peptidyl-threonine phosphorylation [GO:0018107] (BP) Sources: RESID:AA0038 Relationships: is a type of protein phosphorylation [GO:0006468]; is a type of peptidyl-threonine modification [GO:0018210] Subtypes: negative regulation of thioredoxin peroxidase activity by peptidyl-threonine phosphorylation [GO:1903125], peptidyl-threonine autophosphorylation [GO:1990443] Definition: The phosphorylation of peptidyl-threonine to form peptidyl-O-phospho-L-threonine. Regulation: regulated by GO:0010799; positively regulated by GO:0010800; negatively regulated by negative regulation of peptidyl-threonine phosphorylation [GO:0010801]